follicular B cell differentiation [GO:0002316] (biological process) Note: Note that immunologists typically use the word 'development' to refer to cells of B or T cell lineages undergoing the process that GO describes as 'cell differentiation'. Relationships: is a type of GO:0002313 Also known as: follicular B lymphocyte differentiation, follicular B-cell differentiation, follicular B-lymphocyte differentiation, follicular B cell development Sources: GOC:jal, ISBN:0781735149 Definition: The process in which a B cell in the spleen acquires the specialized features of a follicular B cell. Follicular B cells are major population of mature recirculating B cells in the spleen and are located in the B-cell follicle region.